{
  "gene": "UniProtKB:P61024",
  "term_id": "GO:0019901",
  "term_label": "protein kinase binding",
  "gene_symbol": "CKS1B",
  "gene_name": "Cyclin-dependent kinases regulatory subunit 1"
}